{
  "gene": "UniProtKB:O15013",
  "gene_symbol": "ARHGEF10",
  "term_id": "GO:0090307",
  "term_label": "mitotic spindle assembly",
  "gene_name": "Rho guanine nucleotide exchange factor 10"
}